detoxification of nitrogen compound [GO:0051410] (BP) Sources: GOC:ai Definition: Any process that reduces or removes the toxicity of nitrogenous compounds which are dangerous or toxic. This includes the aerobic conversion of toxic compounds to harmless substances. Relationships: is a type of GO:0098754; BFO_0000050 response to nitrogen compound [GO:1901698] Subtypes: indole phytoalexin catabolic process [GO:0046216], bacteriocin catabolic process [GO:0046225], cellular detoxification of nitrogen compound [GO:0070458], gliotoxin catabolic process [GO:2001309] Also known as: detoxification of nitrogenous compound, nitric oxide (NO) detoxification